ketone body metabolic process [GO:1902224] (biological process) Definition: The chemical reactions and pathways involving ketone body. Also known as: ketone body metabolism Subtypes: acetoacetic acid metabolic process [GO:0043438], ketone body biosynthetic process [GO:0046951], GO:0046952 Sources: GOC:TermGenie, GOC:pr Relationships: is a type of generation of precursor metabolites and energy [GO:0006091]; is a type of small molecule metabolic process [GO:0044281]; is a type of fatty acid derivative metabolic process [GO:1901568]